negative regulation of cellular response to oxidative stress [GO:1900408] (biological process) Subtypes: GO:1904832 Sources: GOC:TermGenie, GOC:mah Definition: Any process that stops, prevents or reduces the frequency, rate or extent of cellular response to oxidative stress. Relationships: is a type of GO:0048523; is a type of regulation of cellular response to oxidative stress [GO:1900407]; is a type of GO:1902883; negatively regulates cellular response to oxidative stress [GO:0034599] Also known as: down regulation of cellular response to oxidative stress, down-regulation of cellular response to oxidative stress, downregulation of cellular response to oxidative stress, down regulation of adaptive response to oxidative stress, down-regulation of adaptive response to oxidative stress, downregulation of adaptive response to oxidative stress, inhibition of adaptive response to oxidative stress, inhibition of cellular response to oxidative stress, negative regulation of adaptive response to oxidative stress